rapid tRNA decay [GO:0180037] (biological process) References: PMID:35901126 Sources: GOC:vw Relationships: is a type of tRNA surveillance [GO:0106354] Definition: A cytoplasmic tRNA surveillance pathway that targets mature hypomodified tRNAs, catalyzed by 5'-3' exonucleases Xrn1 (S. cerevisiae/human) and Rat1 (S. cerevisiae) XRN2 human, and regulated by adenosine 3',5' bisphosphate (pAp).